2-ketobutyrate formate-lyase activity [GO:0043875] (molecular function) Also known as: keto-acid formate acetyltransferase, KFL, TdcE Relationships: is a type of acyltransferase activity, transferring groups other than amino-acyl groups [GO:0016747] Note: This function is part of an anaerobic pathway for the catabolism of L-threonine. Definition: Catalysis of the reaction: 2-oxobutanoate + coenzyme A = propionyl-CoA + formate. References: PMID:9484901 Sources: RHEA:28054